{
  "term_id": "GO:0005886",
  "gene_symbol": "DGKB",
  "gene": "UniProtKB:Q9Y6T7",
  "gene_name": "Diacylglycerol kinase beta",
  "term_label": "plasma membrane"
}